protein localization to cortical endoplasmic reticulum [GO:1903419] (biological process) Also known as: protein localisation in cortical endoplasmic reticulum, protein localisation to cortical endoplasmic reticulum, protein localization in cortical endoplasmic reticulum, protein localization to cortical ER References: PMID:25103238 Sources: GOC:TermGenie, GO_REF:0000087 Relationships: is a type of GO:0072697; is_a protein localization to endoplasmic reticulum tubular network [GO:1903420] Definition: A process in which a protein is transported to, or maintained in, a location within a cortical endoplasmic reticulum.